{
  "gene_name": "Mitochondrial coenzyme A diphosphatase NUDT8",
  "gene_symbol": "NUDT8",
  "term_label": "mitochondrion",
  "term_id": "GO:0005739",
  "gene": "UniProtKB:Q8WV74"
}